{
  "gene_name": "Myogenic factor 6",
  "term_id": "GO:0048743",
  "term_label": "positive regulation of skeletal muscle fiber development",
  "gene_symbol": "MYF6",
  "gene": "UniProtKB:P23409"
}